{
  "gene_name": "von Willebrand factor D and EGF domain-containing protein",
  "term_label": "cell surface",
  "gene": "UniProtKB:Q8N2E2",
  "gene_symbol": "VWDE",
  "term_id": "GO:0009986"
}